{
  "gene_symbol": "MYF6",
  "term_id": "GO:0035914",
  "gene_name": "Myogenic factor 6",
  "term_label": "skeletal muscle cell differentiation",
  "gene": "UniProtKB:P23409"
}